{
  "term_label": "Mpp10 complex",
  "term_id": "GO:0034457",
  "gene_name": "U3 small nucleolar ribonucleoprotein protein MPP10",
  "gene": "UniProtKB:O00566",
  "gene_symbol": "MPHOSPH10"
}